negative regulation of maintenance of mitotic sister chromatid cohesion, telomeric [GO:1904908] (biological process) References: PMID:26373281 Sources: GOC:BHF, GOC:BHF_telomere, GOC:TermGenie, GOC:rph, GO_REF:0000058 Definition: Any process that stops, prevents or reduces the frequency, rate or extent of maintenance of mitotic sister chromatid cohesion, telomeric. Relationships: is a type of GO:0034183; is a type of GO:1904907; negatively regulates GO:0099403 Also known as: down regulation of maintenance of mitotic sister chromatid cohesion, telomeric, down regulation of maintenance of mitotic sister chromatin cohesion at telomere, down regulation of maintenance of sister chromatin cohesion at telomere at mitosis, down regulation of maintenance of telomeric mitotic sister chromatin cohesion, down-regulation of maintenance of mitotic sister chromatid cohesion, telomeric, down-regulation of maintenance of mitotic sister chromatin cohesion at telomere, down-regulation of maintenance of sister chromatin cohesion at telomere at mitosis, down-regulation of maintenance of telomeric mitotic sister chromatin cohesion, downregulation of maintenance of mitotic sister chromatid cohesion, telomeric, downregulation of maintenance of mitotic sister chromatin cohesion at telomere, downregulation of maintenance of sister chromatin cohesion at telomere at mitosis, downregulation of maintenance of telomeric mitotic sister chromatin cohesion, negative regulation of maintenance of mitotic sister chromatin cohesion at telomere, negative regulation of maintenance of sister chromatin cohesion at telomere at mitosis, negative regulation of maintenance of telomeric mitotic sister chromatin cohesion, inhibition of maintenance of mitotic sister chromatid cohesion, telomeric, inhibition of maintenance of mitotic sister chromatin cohesion at telomere, inhibition of maintenance of sister chromatin cohesion at telomere at mitosis, inhibition of maintenance of telomeric mitotic sister chromatin cohesion